lead ion binding [GO:0032791] (molecular function) Relationships: is a type of metal ion binding [GO:0046872] Sources: GOC:mah Definition: Binding to lead (Pb) ions.